{
  "term_id": "GO:0003823",
  "gene_symbol": "IGHV2-26",
  "term_label": "antigen binding",
  "gene_name": "Immunoglobulin heavy variable 2-26",
  "gene": "UniProtKB:A0A0B4J1V2"
}